{
  "term_label": "cilium assembly",
  "term_id": "GO:0060271",
  "gene_symbol": "CEP131",
  "gene": "UniProtKB:Q9UPN4",
  "gene_name": "Centrosomal protein of 131 kDa"
}